ovary septum development [GO:0080126] (biological process) Relationships: is a type of developmental process involved in reproduction [GO:0003006]; is_a plant septum development [GO:1905328]; is part of plant-type ovary development [GO:0035670] Definition: The process whose specific outcome is the progression of the ovary septum over time, from its formation to the mature structure. The ovary septum is the thin partition that divides the ovary, the basal portion of a carpel or group of fused carpels, that encloses the ovule(s). References: PMID:17855426